{
  "gene_name": "Zinc finger and BTB domain-containing protein 45",
  "gene_symbol": "ZBTB45",
  "gene": "UniProtKB:Q96K62",
  "term_id": "GO:0005654",
  "term_label": "nucleoplasm"
}